{
  "term_label": "cellular response to growth factor stimulus",
  "gene": "UniProtKB:P27037",
  "term_id": "GO:0071363",
  "gene_name": "Activin receptor type-2A",
  "gene_symbol": "ACVR2A"
}